{
  "term_id": "GO:0006654",
  "gene": "UniProtKB:Q9Y6T7",
  "gene_symbol": "DGKB",
  "gene_name": "Diacylglycerol kinase beta",
  "term_label": "phosphatidic acid biosynthetic process"
}